{
  "gene_name": "Laminin subunit beta-4",
  "gene": "UniProtKB:A4D0S4",
  "gene_symbol": "LAMB4",
  "term_id": "GO:0005201",
  "term_label": "extracellular matrix structural constituent"
}